{
  "term_label": "nuclear envelope",
  "gene_symbol": "CHMP4C",
  "term_id": "GO:0005635",
  "gene_name": "Charged multivesicular body protein 4c",
  "gene": "UniProtKB:Q96CF2"
}